{
  "term_id": "UNKNOWN:0003",
  "term_label": "Unknown cellular component",
  "gene_name": "Dipeptidyl peptidase 9",
  "gene": "UniProtKB:Q86TI2",
  "gene_symbol": "DPP9"
}